{
  "gene": "UniProtKB:A6NP11",
  "gene_symbol": "ZNF716",
  "gene_name": "Zinc finger protein 716",
  "term_id": "UNKNOWN:0003",
  "term_label": "Unknown cellular component"
}